1,4-lactonase activity [GO:0050490] (molecular function) Definition: Catalysis of the reaction: H2O + a 1,4-lactone = a 4-hydroxyacid. Sources: EC:3.1.1.25, MetaCyc:14-LACTONASE-RXN Relationships: is a type of carboxylic ester hydrolase activity [GO:0052689] Also known as: 1,4-lactone hydroxyacylhydrolase activity, gamma-lactonase activity